{
  "gene_name": "Integrin beta-2",
  "term_label": "cell-matrix adhesion",
  "gene_symbol": "ITGB2",
  "term_id": "GO:0007160",
  "gene": "UniProtKB:P05107"
}